{
  "gene_symbol": "ZC3H3",
  "gene_name": "Zinc finger CCCH domain-containing protein 3",
  "term_label": "Unknown molecular function",
  "term_id": "UNKNOWN:0001",
  "gene": "UniProtKB:Q8IXZ2"
}